{
  "gene": "UniProtKB:Q9NX08",
  "gene_symbol": "COMMD8",
  "term_label": "NF-kappaB binding",
  "term_id": "GO:0051059",
  "gene_name": "COMM domain-containing protein 8"
}